{
  "gene": "UniProtKB:Q8NG68",
  "gene_symbol": "TTL",
  "term_label": "spindle microtubule",
  "gene_name": "Tubulin--tyrosine ligase",
  "term_id": "GO:0005876"
}